{
  "gene_symbol": "FLOT2",
  "term_id": "GO:0005886",
  "gene": "UniProtKB:Q14254",
  "term_label": "plasma membrane",
  "gene_name": "Flotillin-2"
}